negative regulation of antipodal cell differentiation [GO:0045689] (biological process) Sources: GOC:go_curators, GOC:mtg_plant Also known as: down regulation of antipodal cell differentiation, down-regulation of antipodal cell differentiation, downregulation of antipodal cell differentiation, inhibition of antipodal cell differentiation Definition: Any process that stops, prevents, or reduces the frequency, rate or extent of antipodal cell differentiation. Relationships: is a type of GO:0045596; is a type of GO:0045688; negatively regulates antipodal cell differentiation [GO:0009557]